glycosphingolipid deacylase activity [GO:0033964] (MF) Also known as: glycosphingolipid ceramide deacylase activity, glycosphingolipid amidohydrolase activity Definition: Catalysis of the hydrolysis of gangliosides and neutral glycosphingolipids, releasing fatty acids to form the lyso-derivatives. Sources: EC:3.5.1.69 Relationships: is a type of hydrolase activity, acting on carbon-nitrogen (but not peptide) bonds, in linear amides [GO:0016811]